{
  "gene_symbol": "IL1R2",
  "term_id": "GO:0004908",
  "gene_name": "Interleukin-1 receptor type 2",
  "term_label": "interleukin-1 receptor activity",
  "gene": "UniProtKB:P27930"
}